{
  "term_id": "GO:0005813",
  "gene_name": "Leucine-rich repeat and coiled-coil domain-containing protein 1",
  "gene_symbol": "LRRCC1",
  "gene": "UniProtKB:Q9C099",
  "term_label": "centrosome"
}